{
  "gene_name": "Apelin receptor early endogenous ligand",
  "gene": "UniProtKB:P0DMC3",
  "term_label": "apelin receptor signaling pathway",
  "term_id": "GO:0060183",
  "gene_symbol": "APELA"
}